{
  "gene_name": "Golgin subfamily A member 6-like protein 26",
  "gene_symbol": "GOLGA6L26",
  "term_label": "Unknown cellular component",
  "gene": "UniProtKB:P0DX02",
  "term_id": "UNKNOWN:0003"
}